{
  "gene_name": "Cyclin-dependent kinase 10",
  "term_label": "G2/M transition of mitotic cell cycle",
  "gene_symbol": "CDK10",
  "term_id": "GO:0000086",
  "gene": "UniProtKB:Q15131"
}